{
  "gene_symbol": "PLEKHA2",
  "term_label": "cytoplasm",
  "gene_name": "Pleckstrin homology domain-containing family A member 2",
  "term_id": "GO:0005737",
  "gene": "UniProtKB:Q9HB19"
}